regulation of insulin receptor signaling pathway [GO:0046626] (BP) Relationships: is a type of GO:0009966; regulates insulin receptor signaling pathway [GO:0008286] Definition: Any process that modulates the frequency, rate or extent of insulin receptor signaling. Sources: GOC:bf Subtypes: negative regulation of insulin receptor signaling pathway [GO:0046627], positive regulation of insulin receptor signaling pathway [GO:0046628] Also known as: regulation of insulin receptor signalling pathway